{
  "gene_name": "Semaphorin-3E",
  "gene": "UniProtKB:O15041",
  "term_id": "GO:0005615",
  "gene_symbol": "SEMA3E",
  "term_label": "extracellular space"
}